cAMP binding [GO:0030552] (molecular function) Definition: Binding to cAMP, the nucleotide cyclic AMP (adenosine 3',5'-cyclophosphate). Relationships: is a type of cyclic nucleotide binding [GO:0030551]; is a type of adenyl ribonucleotide binding [GO:0032559]; is a type of anion binding [GO:0043168] Also known as: 3',5' cAMP binding, 3',5'-cAMP binding, adenosine 3',5'-cyclophosphate binding, cyclic AMP binding Sources: GOC:ai